{
  "gene_symbol": "USP54",
  "gene": "UniProtKB:Q70EL1",
  "gene_name": "Inactive ubiquitin carboxyl-terminal hydrolase 54",
  "term_id": "UNKNOWN:0001",
  "term_label": "Unknown molecular function"
}